{
  "term_id": "GO:0008569",
  "term_label": "minus-end-directed microtubule motor activity",
  "gene_symbol": "DNAH10",
  "gene_name": "Dynein axonemal heavy chain 10",
  "gene": "UniProtKB:Q8IVF4"
}